{
  "gene_symbol": "IGF1",
  "gene": "UniProtKB:P05019",
  "term_label": "positive regulation of phosphatidylinositol 3-kinase/protein kinase B signal transduction",
  "term_id": "GO:0051897",
  "gene_name": "Insulin-like growth factor I"
}